{
  "gene_symbol": "RHO",
  "term_label": "G protein-coupled photoreceptor activity",
  "gene_name": "Rhodopsin",
  "gene": "UniProtKB:P08100",
  "term_id": "GO:0008020"
}